decaprenyl-N-acetyl-alpha-D-glucosaminyl-pyrophosphate:dTDP-alpha-L-rhamnose rhamnosyltransferase activity [GO:0102096] (molecular function) Sources: EC:2.4.1.289, GOC:pz Relationships: is_a hexosyltransferase activity [GO:0016758] Definition: Catalysis of the reaction: dTDP-6-deoxy-beta-L-mannose + N-acetyl-alpha-D-glucosaminyl-diphospho-trans,octacis-decaprenol = dTDP(3-) + alpha-L-Rhap-(1->3)-alpha-D-GlcpNAc-1-diphospho-trans,octacis-decaprenol + H+.